{
  "term_id": "GO:0006182",
  "term_label": "cGMP biosynthetic process",
  "gene_symbol": "GUCY1B1",
  "gene_name": "Guanylate cyclase soluble subunit beta-1",
  "gene": "UniProtKB:Q02153"
}